{
  "gene_symbol": "COBLL1",
  "term_id": "UNKNOWN:0003",
  "term_label": "Unknown cellular component",
  "gene": "UniProtKB:Q53SF7",
  "gene_name": "Cordon-bleu protein-like 1"
}